high-affinity ferric iron transmembrane transporter activity [GO:0015092] (molecular function) Also known as: high affinity ferric uptake transmembrane transporter activity Relationships: is a type of ferric iron transmembrane transporter activity [GO:0015091] References: PMID:1447137 Sources: GOC:ai Definition: Enables the transfer of ferric iron (Fe(III) or Fe3+) ions from one side of a membrane to the other. In high-affinity transport the transporter is able to bind the solute even if it is only present at very low concentrations.